{
  "gene": "UniProtKB:A6NMK7",
  "gene_symbol": "CPSF4L",
  "gene_name": "Putative cleavage and polyadenylation specificity factor subunit 4-like protein",
  "term_label": "mRNA cleavage and polyadenylation specificity factor complex",
  "term_id": "GO:0005847"
}